{
  "gene_symbol": "SKOR2",
  "gene_name": "SKI family transcriptional corepressor 2",
  "term_id": "GO:0046332",
  "gene": "UniProtKB:Q2VWA4",
  "term_label": "SMAD binding"
}